{
  "gene": "UniProtKB:Q03060",
  "term_label": "DNA-binding transcription factor activity, RNA polymerase II-specific",
  "gene_name": "cAMP-responsive element modulator",
  "gene_symbol": "CREM",
  "term_id": "GO:0000981"
}